{
  "gene": "UniProtKB:Q9UPW8",
  "gene_symbol": "UNC13A",
  "gene_name": "Protein unc-13 homolog A",
  "term_label": "presynaptic membrane",
  "term_id": "GO:0042734"
}